D-lactate dehydrogenase activity [GO:0047809] (molecular function) Subtypes: D-lactate dehydrogenase (cytochrome) activity [GO:0004458], GO:0008720, D-lactate dehydrogenase (quinone) activity [GO:0102029], GO:0140170 Also known as: D-2-hydroxy-acid dehydrogenase activity, (R)-lactate dehydrogenase activity, (R)-2-hydroxy-acid:(acceptor) 2-oxidoreductase activity, 2-hydroxy acid dehydrogenase activity Definition: Catalysis of the reaction: (R)-lactate + A = AH(2) + pyruvate. Sources: RHEA:15089 Relationships: is a type of GO:0004457; is a type of (2R)-oxo-acid reductase activity [GO:0033719]